{
  "gene": "UniProtKB:Q9NQV7",
  "gene_name": "Histone-lysine N-methyltransferase PRDM9",
  "term_id": "GO:0010468",
  "gene_symbol": "PRDM9",
  "term_label": "regulation of gene expression"
}